{
  "term_label": "Unknown molecular function",
  "gene": "UniProtKB:Q7Z3T8",
  "term_id": "UNKNOWN:0001",
  "gene_name": "Zinc finger FYVE domain-containing protein 16",
  "gene_symbol": "ZFYVE16"
}